{
  "term_id": "GO:0070064",
  "gene": "UniProtKB:Q9H706",
  "gene_symbol": "GAREM1",
  "gene_name": "GRB2-associated and regulator of MAPK protein 1",
  "term_label": "proline-rich region binding"
}